{
  "gene": "UniProtKB:Q8NEZ4",
  "term_id": "GO:0044666",
  "gene_name": "Histone-lysine N-methyltransferase 2C",
  "term_label": "MLL3/4 complex",
  "gene_symbol": "KMT2C"
}